glycine-gated cation channel activity [GO:0160212] (molecular function) References: PMID:11823786 Definition: Enables the transmembrane transfer of a cation by a channel that opens when glycine is bound by the channel complex or one of its constituent parts on the extracellular side of the plasma membrane. Relationships: is a type of GO:0022824; is a type of ligand-gated monoatomic cation channel activity [GO:0099094]